{
  "gene_symbol": "SKA2",
  "term_id": "GO:0005876",
  "gene_name": "Spindle and kinetochore-associated protein 2",
  "gene": "UniProtKB:Q8WVK7",
  "term_label": "spindle microtubule"
}